{
  "gene_name": "PRAME family member 11",
  "gene_symbol": "PRAMEF11",
  "gene": "UniProtKB:O60813",
  "term_label": "proteasome-mediated ubiquitin-dependent protein catabolic process",
  "term_id": "GO:0043161"
}